{
  "gene_name": "Pancreatic lipase-related protein 3",
  "term_label": "triglyceride catabolic process",
  "gene_symbol": "PNLIPRP3",
  "gene": "UniProtKB:Q17RR3",
  "term_id": "GO:0019433"
}